regulation of ribonuclease activity [GO:0060700] (biological process) Subtypes: regulation of endoribonuclease activity [GO:0060699] Sources: GOC:dph, GOC:tb Relationships: is a type of regulation of catalytic activity [GO:0050790]; is a type of regulation of RNA metabolic process [GO:0051252]; regulates RNA nuclease activity [GO:0004540] Definition: Any process that modulates the rate, frequency, or extent of ribonuclease activity, catalysis of the hydrolysis of phosphodiester bonds in chains of RNA.